{
  "gene_symbol": "KIN",
  "gene_name": "DNA_RNA-binding protein KIN17",
  "gene": "UniProtKB:O60870",
  "term_label": "DNA damage response",
  "term_id": "GO:0006974"
}